{
  "term_id": "GO:0022011",
  "gene": "UniProtKB:Q8N135",
  "gene_symbol": "LGI4",
  "gene_name": "Leucine-rich repeat LGI family member 4",
  "term_label": "myelination in peripheral nervous system"
}